{
  "gene": "UniProtKB:Q9UPY5",
  "gene_name": "Cystine_glutamate transporter",
  "term_label": "L-amino acid transmembrane transporter activity",
  "gene_symbol": "SLC7A11",
  "term_id": "GO:0015179"
}